regulation of oskar mRNA translation [GO:0046011] (biological process) References: PMID:12538512 Sources: GOC:go_curators Relationships: is a type of regulation of translation [GO:0006417] Subtypes: negative regulation of oskar mRNA translation [GO:0007319], positive regulation of oskar mRNA translation [GO:0046012] Definition: Any process that modulates the frequency, rate or extent of oskar mRNA translation. To ensure the localization of Oskar protein at the posterior pole of the oocyte, translation of oskar mRNA is repressed during its transport to the posterior pole and activated upon localization of the mRNA at the posterior cortex.